{
  "gene_symbol": "CD84",
  "term_label": "external side of plasma membrane",
  "gene": "UniProtKB:Q9UIB8",
  "term_id": "GO:0009897",
  "gene_name": "SLAM family member 5"
}